{
  "term_id": "GO:0005832",
  "gene_symbol": "CCT8L2",
  "term_label": "chaperonin-containing T-complex",
  "gene_name": "T-complex protein 1 subunit theta-like 2",
  "gene": "UniProtKB:Q96SF2"
}